{
  "term_id": "UNKNOWN:0001",
  "gene_symbol": "LRFN3",
  "term_label": "Unknown molecular function",
  "gene": "UniProtKB:Q9BTN0",
  "gene_name": "Leucine-rich repeat and fibronectin type-III domain-containing protein 3"
}